group II metabotropic glutamate receptor activity [GO:0001641] (molecular function) Definition: A G protein-coupled receptor that is activated by trans-1-aminocyclopentane-1,3-dicarboxylic acid (t-ACPD) and inhibits adenylate cyclase activity. Sources: GOC:dph Relationships: is a type of adenylate cyclase inhibiting G protein-coupled glutamate receptor activity [GO:0001640]